{
  "term_label": "integrin-mediated signaling pathway",
  "gene_name": "Integrin alpha-9",
  "gene": "UniProtKB:Q13797",
  "gene_symbol": "ITGA9",
  "term_id": "GO:0007229"
}